{
  "gene": "UniProtKB:Q9BV38",
  "term_id": "GO:0006261",
  "term_label": "DNA-templated DNA replication",
  "gene_name": "WD repeat-containing protein 18",
  "gene_symbol": "WDR18"
}